{
  "term_id": "GO:0005829",
  "term_label": "cytosol",
  "gene": "UniProtKB:P30048",
  "gene_name": "Thioredoxin-dependent peroxide reductase, mitochondrial",
  "gene_symbol": "PRDX3"
}